{
  "gene_symbol": "RPS6KL1",
  "gene_name": "Ribosomal protein S6 kinase-like 1",
  "gene": "UniProtKB:Q9Y6S9",
  "term_label": "Unknown biological process",
  "term_id": "UNKNOWN:0002"
}